6-oxohexanoate dehydrogenase activity [GO:0018483] (molecular function) Sources: EC:1.2.1.63 Relationships: is a type of GO:0016620 Definition: Catalysis of the reaction: 6-oxohexanoate + NADP+ + H2O = adipate + NADPH + H+. Also known as: 6-oxohexanoate:NADP+ oxidoreductase activity